{
  "gene_symbol": "QSOX1",
  "gene": "UniProtKB:O00391",
  "term_id": "GO:0003756",
  "gene_name": "Sulfhydryl oxidase 1",
  "term_label": "protein disulfide isomerase activity"
}